{
  "term_id": "GO:0007411",
  "gene_name": "Basigin",
  "gene_symbol": "BSG",
  "gene": "UniProtKB:P35613",
  "term_label": "axon guidance"
}